{
  "gene": "UniProtKB:A4D0V7",
  "gene_symbol": "CPED1",
  "term_label": "Unknown molecular function",
  "term_id": "UNKNOWN:0001",
  "gene_name": "Cadherin-like and PC-esterase domain-containing protein 1"
}